apolipoprotein receptor activity [GO:0030226] (molecular function) Sources: GOC:mah, ISBN:0198506732 Relationships: is_a GO:0038024; has part apolipoprotein binding [GO:0034185] Subtypes: apolipoprotein A-I receptor activity [GO:0034188] Definition: Combining with an apolipoprotein to initiate a change in cell activity.